transcription export complex [GO:0000346] (cellular component) Also known as: TREX complex Definition: The transcription export (TREX) complex couples transcription elongation by RNA polymerase II to mRNA export. The complex associates with the polymerase and travels with it along the length of the transcribed gene. TREX is composed of the THO transcription elongation complex as well as other proteins that couple THO to mRNA export proteins. The TREX complex is known to be found in a wide range of eukaryotes, including S. cerevisiae and metazoans. Relationships: is a type of nuclear protein-containing complex [GO:0140513] References: PMID:11979277 Sources: GOC:krc